M band [GO:0031430] (cellular component) Definition: The midline of aligned thick filaments in a sarcomere; location of specific proteins that link thick filaments. Depending on muscle type the M band consists of different numbers of M lines. Sources: GOC:mtg_muscle, ISBN:0198506732, ISBN:0815316194 Also known as: midline, M disc, mesophragma, M line Relationships: is a type of GO:0110165; is part of A band [GO:0031672]